PML body organization [GO:0030578] (biological process) Definition: A process that is carried out at the cellular level which results in the assembly, arrangement of constituent parts, or disassembly of PML bodies, a class of nuclear body; they react against SP100 auto-antibodies (PML = promyelocytic leukemia). Note: See also the cellular component term 'PML body ; GO:0016605'. Also known as: PML body organisation, PML body organization and biogenesis Relationships: is a type of nuclear body organization [GO:0030575] References: PMID:10806078 Sources: GOC:mah